{
  "gene_name": "Proton-coupled amino acid transporter 1",
  "gene_symbol": "SLC36A1",
  "term_label": "proline transmembrane transport",
  "gene": "UniProtKB:Q7Z2H8",
  "term_id": "GO:0035524"
}